{
  "gene_symbol": "TEX22",
  "term_label": "Unknown molecular function",
  "gene": "UniProtKB:C9J3V5",
  "gene_name": "Testis-expressed protein 22",
  "term_id": "UNKNOWN:0001"
}